{
  "term_id": "GO:0034142",
  "term_label": "toll-like receptor 4 signaling pathway",
  "gene_symbol": "MYD88",
  "gene_name": "Myeloid differentiation primary response protein MyD88",
  "gene": "UniProtKB:Q99836"
}